{
  "term_label": "kinetochore",
  "term_id": "GO:0000776",
  "gene": "UniProtKB:Q9GZM8",
  "gene_symbol": "NDEL1",
  "gene_name": "Nuclear distribution protein nudE-like 1"
}